{
  "gene": "UniProtKB:O75159",
  "gene_symbol": "SOCS5",
  "term_id": "UNKNOWN:0003",
  "term_label": "Unknown cellular component",
  "gene_name": "Suppressor of cytokine signaling 5"
}